{
  "gene": "UniProtKB:O75146",
  "term_id": "GO:2000588",
  "gene_symbol": "HIP1R",
  "term_label": "positive regulation of platelet-derived growth factor receptor-beta signaling pathway",
  "gene_name": "Huntingtin-interacting protein 1-related protein"
}